mesonephric glomerular mesangial cell development [GO:0061263] (biological process) Sources: GOC:mtg_kidney_jan10 Relationships: is a type of GO:0072144; is part of GO:0061259 Definition: The process whose specific outcome is the progression of a glomerular mesangial cell in the mesonephros over time, from its formation to the mature structure.